neuronal dense core vesicle [GO:0098992] (cellular component) Relationships: is a type of dense core granule [GO:0031045] Sources: GOC:dos, ISBN:978-0-07-181001-2, Wikipedia:Neuropeptide&oldid=713905176 Definition: A dense core vesicle (granule) that is part of a neuron. These vesicles typically contain neuropeptides. They can be found in all parts of neurons, including the soma, dendrites, axonal swellings (varicosities) and synaptic terminals.